{
  "gene_symbol": "ANKRD10",
  "term_id": "UNKNOWN:0002",
  "term_label": "Unknown biological process",
  "gene": "UniProtKB:Q9NXR5",
  "gene_name": "Ankyrin repeat domain-containing protein 10"
}